{
  "gene_symbol": "VPS13D",
  "term_id": "UNKNOWN:0001",
  "term_label": "Unknown molecular function",
  "gene": "UniProtKB:Q5THJ4",
  "gene_name": "Intermembrane lipid transfer protein VPS13D"
}